haltere disc development [GO:0035216] (biological process) Definition: Progression of the haltere imaginal disc over time, from its initial formation through to its metamorphosis to form the adult capitellum, pedicel, haltere sclerite, metathoracic spiracle and metanotum. Relationships: is a type of imaginal disc development [GO:0007444] Sources: GOC:bf, ISBN:0879694238